lipid exchange activity [GO:7770011] (molecular function) Definition: Enables the transfer of a specific lipid molecule from one membrane to another, coupled with the simultaneous counter-transfer of a different lipid molecule in the opposite direction. References: PMID:32793602 Relationships: is_a lipid transfer activity [GO:0120013] Subtypes: phosphatidylserine-phosphatidylinositol-4-phosphate exchange activity [GO:0160270], phosphatidylinositol-4-phosphate-cholesterol exchange activity [GO:0160291]